{
  "gene": "UniProtKB:Q8WVZ9",
  "term_label": "proteasome-mediated ubiquitin-dependent protein catabolic process",
  "gene_symbol": "KBTBD7",
  "gene_name": "Kelch repeat and BTB domain-containing protein 7",
  "term_id": "GO:0043161"
}